{
  "term_label": "Unknown biological process",
  "term_id": "UNKNOWN:0002",
  "gene_symbol": "CCER1",
  "gene": "UniProtKB:Q8TC90",
  "gene_name": "Coiled-coil domain-containing glutamate-rich protein 1"
}